xylulose metabolic process [GO:0005997] (biological process) Subtypes: xylulose catabolic process [GO:0005998], xylulose biosynthetic process [GO:0005999] Also known as: xylulose metabolism Sources: ISBN:0198547684 Relationships: is a type of pentose metabolic process [GO:0019321] Definition: The chemical reactions and pathways involving xylulose, the ketopentose threo-2-pentulose.